regulation of cell wall (1->3)-beta-D-glucan biosynthetic process [GO:0090334] (biological process) Definition: Any process that modulates the rate, frequency, or extent of the chemical reactions and pathways resulting in the formation of (1->3)-beta-D-glucans, compounds composed of glucose residues linked by (1->3)-beta-D-glucosidic bonds, found in the walls of cells. Sources: GOC:tb Relationships: is a type of regulation of cell wall macromolecule metabolic process [GO:0010981]; is a type of GO:0032953; is a type of GO:1903338; regulates cell wall (1->3)-beta-D-glucan biosynthetic process [GO:0034411] Also known as: regulation of cell wall 1,3-beta-D-glucan biosynthetic process, regulation of cell wall 1,3-beta-glucan biosynthetic process Subtypes: regulation of ascospore wall (1->3)-beta-D-glucan biosynthetic process [GO:0060624]